regulation of T-helper 1 type immune response [GO:0002825] (biological process) Subtypes: negative regulation of T-helper 1 type immune response [GO:0002826], positive regulation of T-helper 1 type immune response [GO:0002827], regulation of T-helper 1 cell differentiation [GO:0045625], regulation of T-helper 1 cell cytokine production [GO:2000554] Relationships: is a type of regulation of adaptive immune response based on somatic recombination of immune receptors built from immunoglobulin superfamily domains [GO:0002822]; regulates T-helper 1 type immune response [GO:0042088] Sources: GOC:add Definition: Any process that modulates the frequency, rate, or extent of a T-helper 1 type immune response.